{
  "term_label": "actin filament binding",
  "gene_symbol": "CNN1",
  "term_id": "GO:0051015",
  "gene": "UniProtKB:P51911",
  "gene_name": "Calponin-1"
}